{
  "gene_symbol": "POLQ",
  "gene_name": "DNA polymerase theta",
  "gene": "UniProtKB:O75417",
  "term_label": "DNA-directed DNA polymerase activity",
  "term_id": "GO:0003887"
}